{
  "term_label": "acrosomal vesicle",
  "term_id": "GO:0001669",
  "gene": "UniProtKB:Q8NA54",
  "gene_symbol": "IQUB",
  "gene_name": "IQ and ubiquitin-like domain-containing protein"
}